transcription initiation at RNA polymerase I promoter [GO:0006361] (biological process) Note: Note that promoter clearance is represented as a separate step, not part_of either initiation or elongation. Sources: GOC:txnOH Also known as: transcription initiation from Pol I promoter, transcription initiation from RNA polymerase I promoter, transcription initiation from RNA polymerase I promoter for nuclear large rRNA transcript Definition: A transcription initiation process that takes place at a RNA polymerase I gene promoter. Ribosomal RNAs (rRNA) genes are transcribed by RNA polymerase I. Regulation: regulated by regulation of transcription initiation by RNA polymerase I [GO:1903357] Relationships: is a type of GO:0006352; is part of transcription by RNA polymerase I [GO:0006360]